{
  "gene_symbol": "SCGB1D1",
  "term_label": "extracellular space",
  "term_id": "GO:0005615",
  "gene": "UniProtKB:O95968",
  "gene_name": "Secretoglobin family 1D member 1"
}